{
  "gene_name": "Tudor domain-containing protein 1",
  "gene": "UniProtKB:Q9BXT4",
  "term_label": "piRNA processing",
  "gene_symbol": "TDRD1",
  "term_id": "GO:0034587"
}